mitochondrial RNA processing [GO:0000963] (biological process) Sources: GOC:krc, GOC:mah Subtypes: GO:0000964, GO:0000965, mitochondrial mRNA processing [GO:0090615], mitochondrial tRNA processing [GO:0090646], mitochondrial mRNA polyadenylation [GO:0097222], mitochondrial polycistronic RNA processing [GO:0140040] Relationships: is a type of RNA processing [GO:0006396]; is a type of mitochondrial gene expression [GO:0140053]; BFO_0000050 mitochondrial RNA metabolic process [GO:0000959] Definition: The conversion of a primary RNA molecule transcribed from a mitochondrial genome into one or more mature RNA molecules; occurs in the mitochondrion.